smooth muscle cell-matrix adhesion [GO:0061302] (biological process) Regulation: positively regulated by positive regulation of smooth muscle cell-matrix adhesion [GO:1905609]; RO_0002211 by GO:2000097; negatively regulated by negative regulation of smooth muscle cell-matrix adhesion [GO:2000098] References: PMID:8837777 Sources: GOC:BHF, GOC:dph Relationships: is a type of cell-matrix adhesion [GO:0007160] Definition: The binding of a smooth muscle cell to the extracellular matrix via adhesion molecules.